phosphatidylinositol-3-phosphate phosphatase activity [GO:0004438] (molecular function) Note: Note that this function includes EC:3.1.3.65. Sources: EC:3.1.3.64 Also known as: phosphatidylinositol-3-phosphatase activity, 1-phosphatidyl-1D-myo-inositol-3-phosphate 3-phosphohydrolase activity, D-myo-inositol-1,3-bisphosphate 3-phosphohydrolase activity, inositol 1,3-bisphosphate phosphatase activity, inositol-1,3-bisphosphate 3-phosphatase activity, inositol-polyphosphate 3-phosphatase activity, phosphatidyl-3-phosphate 3-phosphohydrolase activity Definition: Catalysis of the reaction: 1-phosphatidyl-1D-myo-inositol 3-phosphate + H2O = 1-phosphatidyl-1D-myo-inositol + phosphate. Relationships: is a type of phosphatidylinositol monophosphate phosphatase activity [GO:0052744]